{
  "gene_name": "UBX domain-containing protein 10",
  "term_label": "endoplasmic reticulum",
  "term_id": "GO:0005783",
  "gene_symbol": "UBXN10",
  "gene": "UniProtKB:Q96LJ8"
}